neuroblast differentiation [GO:0014016] (biological process) Subtypes: forebrain neuroblast differentiation [GO:0021863] Sources: GOC:ef, ISBN:0878932585 Relationships: is a type of cell differentiation [GO:0030154]; is part of generation of neurons [GO:0048699] Definition: The process in which a relatively unspecialized cell acquires specialized features of a neuroblast. There are at least four stages through which the pluripotent cells of epiblast or blastula become neuroblasts.